{
  "gene_name": "HORMA domain-containing protein 2",
  "gene": "UniProtKB:Q8N7B1",
  "term_id": "GO:0051598",
  "term_label": "meiotic recombination checkpoint signaling",
  "gene_symbol": "HORMAD2"
}